{
  "gene": "UniProtKB:Q9NYL4",
  "gene_symbol": "FKBP11",
  "term_label": "peptidyl-prolyl cis-trans isomerase activity",
  "term_id": "GO:0003755",
  "gene_name": "Peptidyl-prolyl cis-trans isomerase FKBP11"
}